{
  "term_id": "GO:0031777",
  "gene_symbol": "PMCH",
  "gene_name": "Pro-MCH",
  "gene": "UniProtKB:P20382",
  "term_label": "type 1 melanin-concentrating hormone receptor binding"
}